{
  "gene_name": "Alkylated DNA repair protein alkB homolog 8",
  "term_label": "tRNA binding",
  "gene_symbol": "ALKBH8",
  "term_id": "GO:0000049",
  "gene": "UniProtKB:Q96BT7"
}